{
  "term_label": "Unknown cellular component",
  "gene_name": "Beta-defensin 116",
  "gene_symbol": "DEFB116",
  "gene": "UniProtKB:Q30KQ4",
  "term_id": "UNKNOWN:0003"
}